{
  "gene_name": "Zinc finger protein 330",
  "term_label": "nucleus",
  "term_id": "GO:0005634",
  "gene": "UniProtKB:Q9Y3S2",
  "gene_symbol": "ZNF330"
}